{
  "term_id": "GO:0003712",
  "gene_name": "Transcription elongation regulator 1-like protein",
  "term_label": "transcription coregulator activity",
  "gene_symbol": "TCERG1L",
  "gene": "UniProtKB:Q5VWI1"
}